{
  "gene_name": "Protein phosphatase 1 regulatory subunit 1A",
  "gene": "UniProtKB:Q13522",
  "gene_symbol": "PPP1R1A",
  "term_id": "GO:0035556",
  "term_label": "intracellular signal transduction"
}